{
  "term_label": "RNA polymerase II cis-regulatory region sequence-specific DNA binding",
  "gene_name": "Zinc finger protein 540",
  "term_id": "GO:0000978",
  "gene": "UniProtKB:Q8NDQ6",
  "gene_symbol": "ZNF540"
}